{
  "term_label": "Unknown cellular component",
  "gene_symbol": "ST6GALNAC2",
  "gene_name": "Alpha-N-acetylgalactosaminide alpha-2,6-sialyltransferase 2",
  "term_id": "UNKNOWN:0003",
  "gene": "UniProtKB:Q9UJ37"
}